regulation of leaf formation [GO:2000025] (biological process) Definition: Any process that modulates the frequency, rate or extent of leaf formation. Relationships: is a type of GO:1905428; regulates leaf formation [GO:0010338] Sources: GOC:obol